{
  "gene_name": "Putative protein PTGES3L",
  "term_id": "GO:0005829",
  "term_label": "cytosol",
  "gene": "UniProtKB:E9PB15",
  "gene_symbol": "PTGES3L"
}